{
  "gene_name": "Protein S100-A14",
  "term_label": "chemokine receptor binding",
  "term_id": "GO:0042379",
  "gene_symbol": "S100A14",
  "gene": "UniProtKB:Q9HCY8"
}